protein-phosphocysteine-D-sorbitol-phosphotransferase system transporter activity [GO:0090583] (molecular function) Definition: Catalysis of the PEP-dependent, phosphoryl transfer-driven transport of substances across a membrane. The transport happens by catalysis of the reaction: protein S-phosphocysteine + D-sorbitol(out) = protein cysteine + D-sorbitol-1-phosphate(in). References: PMID:8875915 Relationships: is a type of protein-phosphocysteine-sugar phosphotransferase activity [GO:0090563]